{
  "gene_symbol": "DNALI1",
  "gene_name": "Axonemal dynein light intermediate polypeptide 1",
  "term_label": "Unknown biological process",
  "term_id": "UNKNOWN:0002",
  "gene": "UniProtKB:O14645"
}